proton-dependent oligopeptide secondary active transmembrane transporter activity [GO:0005427] (molecular function) Definition: Enables the transfer of a oligopeptide from one side of a membrane to the other, up its concentration gradient. The transporter binds the solute and undergoes a series of conformational changes. Transport works equally well in either direction and is driven by proton movement. Also known as: proton-dependent oligopeptide transporter activity, hydrogen/oligopeptide symporter Sources: GOC:mtg_transport, OMIM:600544 Relationships: is a type of GO:0015291